{
  "term_label": "BMP signaling pathway",
  "term_id": "GO:0030509",
  "gene_name": "Protein FAM83G",
  "gene": "UniProtKB:A6ND36",
  "gene_symbol": "FAM83G"
}